{
  "term_id": "UNKNOWN:0002",
  "gene_symbol": "THSD4",
  "gene_name": "Thrombospondin type-1 domain-containing protein 4",
  "gene": "UniProtKB:Q6ZMP0",
  "term_label": "Unknown biological process"
}